N-acetylneuraminate lyase activity [GO:0008747] (molecular function) Relationships: is a type of oxo-acid-lyase activity [GO:0016833] Definition: Catalysis of the reaction: N-acetylneuraminate = N-acetyl-D-mannosamine + pyruvate. Also known as: N-acetylneuraminate aldolase activity, N-acetylneuraminate pyruvate-lyase (N-acetyl-D-mannosamine-forming), N-acetylneuraminate pyruvate-lyase activity, N-acetylneuraminic acid aldolase activity, N-acetylneuraminic acid lyase activity, N-acetylneuraminic aldolase activity, N-acetylneuraminic lyase activity, NALase activity, NANA lyase activity, NPL, acetylneuraminate lyase activity, acetylneuraminate pyruvate-lyase activity, neuraminate aldolase activity, neuraminic acid aldolase activity, neuraminic aldolase activity, sialate lyase activity, sialic acid aldolase activity, sialic aldolase activity Sources: EC:4.1.3.3, RHEA:23296